{
  "term_label": "chromatin",
  "gene_name": "MAU2 chromatid cohesion factor homolog",
  "term_id": "GO:0000785",
  "gene": "UniProtKB:Q9Y6X3",
  "gene_symbol": "MAU2"
}